centriolar subdistal appendage [GO:0120103] (cellular component) Relationships: is a type of GO:0140535; is part of cilium [GO:0005929] Definition: A protein complex which assembles on the mother centriole during cilium formation, adjacent and proximal to a centriolar distal appendage. In human, it contains ODF2, CNTRL, NIN, CCDC120c and CCDC68. Also known as: subdistal appendage of basal body, subdistal appendage of centriole, subdistal appendage of mother centriole References: PMID:23213374, PMID:27818179, PMID:28422092 Sources: GOC:cilia